{
  "gene": "UniProtKB:P78386",
  "term_id": "GO:0045095",
  "gene_name": "Keratin, type II cuticular Hb5",
  "term_label": "keratin filament",
  "gene_symbol": "KRT85"
}